{
  "gene": "UniProtKB:Q8N6C5",
  "term_label": "transmembrane signaling receptor activity",
  "term_id": "GO:0004888",
  "gene_name": "Immunoglobulin superfamily member 1",
  "gene_symbol": "IGSF1"
}